{
  "term_label": "Unknown molecular function",
  "gene_symbol": "BTBD2",
  "term_id": "UNKNOWN:0001",
  "gene": "UniProtKB:Q9BX70",
  "gene_name": "BTB_POZ domain-containing protein 2"
}